{
  "gene_symbol": "GDF11",
  "term_label": "transforming growth factor beta receptor signaling pathway",
  "gene_name": "Growth_differentiation factor 11",
  "gene": "UniProtKB:O95390",
  "term_id": "GO:0007179"
}